BAD-BCL-xl complex [GO:0097137] (CC) Definition: A heterodimeric protein complex consisting of BAD and BCL-xl, members of the Bcl-2 family of anti- and proapoptotic regulators. References: PMID:14634621 Sources: GOC:so Relationships: is a type of GO:0097136